{
  "gene_name": "Proliferation marker protein Ki-67",
  "term_label": "nucleus",
  "term_id": "GO:0005634",
  "gene": "UniProtKB:P46013",
  "gene_symbol": "MKI67"
}